{
  "gene_symbol": "NPAS4",
  "gene": "UniProtKB:Q8IUM7",
  "term_id": "GO:0006357",
  "gene_name": "Neuronal PAS domain-containing protein 4",
  "term_label": "regulation of transcription by RNA polymerase II"
}